DnaA-HU complex [GO:1990103] (cellular component) Definition: A protein-DNA complex containing DNA-bound DnaA attached to HU. HU is a dimer encoded by two closely related genes. Essential for the initiation of replication in bacteria; stimulates the DnaA-dependent unwinding of oriC. References: PMID:18179598 Sources: GOC:bhm Also known as: DnaA-HU-DNA complex Relationships: is_a primosome complex [GO:1990077]